{
  "gene": "UniProtKB:Q8NHL6",
  "gene_symbol": "LILRB1",
  "gene_name": "Leukocyte immunoglobulin-like receptor subfamily B member 1",
  "term_id": "GO:0032396",
  "term_label": "inhibitory MHC class I receptor activity"
}